{
  "term_id": "GO:0005769",
  "gene_symbol": "TBC1D16",
  "gene": "UniProtKB:Q8TBP0",
  "term_label": "early endosome",
  "gene_name": "TBC1 domain family member 16"
}